{
  "gene": "UniProtKB:P42081",
  "term_id": "UNKNOWN:0001",
  "gene_name": "T-lymphocyte activation antigen CD86",
  "gene_symbol": "CD86",
  "term_label": "Unknown molecular function"
}